galactolipid biosynthetic process [GO:0019375] (biological process) Relationships: is a type of glycolipid biosynthetic process [GO:0009247]; is a type of GO:0019374 Also known as: galactolipid anabolism, galactolipid biosynthesis, galactolipid formation, galactolipid synthesis Sources: ISBN:0198506732 Definition: The chemical reactions and pathways resulting in the formation of galactolipids, any glycolipid containing one of more residues of galactose and/or N-acetylgalactosamine. Subtypes: galactosylceramide biosynthetic process [GO:0006682]